{
  "term_id": "GO:0008584",
  "gene_symbol": "ADAM18",
  "gene": "UniProtKB:Q9Y3Q7",
  "term_label": "male gonad development",
  "gene_name": "Disintegrin and metalloproteinase domain-containing protein 18"
}